{
  "gene": "UniProtKB:Q9Y3N9",
  "term_label": "detection of chemical stimulus involved in sensory perception of smell",
  "gene_symbol": "OR2W1",
  "term_id": "GO:0050911",
  "gene_name": "Olfactory receptor 2W1"
}